monocyte chemotaxis [GO:0002548] (biological process) Definition: The movement of a monocyte in response to an external stimulus. References: PMID:11696603, PMID:15173832 Sources: GOC:add Regulation: regulated by regulation of monocyte chemotaxis [GO:0090025]; positively regulated by positive regulation of monocyte chemotaxis [GO:0090026]; RO_0002212 by negative regulation of monocyte chemotaxis [GO:0090027] Relationships: is a type of leukocyte chemotaxis [GO:0030595]; is a type of mononuclear cell migration [GO:0071674]; is a type of myeloid leukocyte migration [GO:0097529]